actinomycete-type spore formation [GO:0034304] (biological process) Relationships: is a type of reproductive process in single-celled organism [GO:0022413]; is a type of asexual sporulation resulting in formation of a cellular spore [GO:0043936] Sources: GOC:ds, ISBN:0122268008 Definition: The process in which differentiated, resting cells are formed from a substrate mycelium; characteristic of many members of the order Actinomycetales.